{
  "gene_symbol": "TMOD4",
  "term_id": "GO:0006936",
  "gene": "UniProtKB:Q9NZQ9",
  "term_label": "muscle contraction",
  "gene_name": "Tropomodulin-4"
}